{
  "gene_symbol": "GPR150",
  "gene_name": "Probable G-protein coupled receptor 150",
  "term_id": "GO:0032870",
  "term_label": "cellular response to hormone stimulus",
  "gene": "UniProtKB:Q8NGU9"
}